{
  "gene_name": "Cadherin-19",
  "term_id": "GO:0005912",
  "term_label": "adherens junction",
  "gene": "UniProtKB:Q9H159",
  "gene_symbol": "CDH19"
}